{
  "gene_symbol": "PDLIM1",
  "gene": "UniProtKB:O00151",
  "term_label": "muscle alpha-actinin binding",
  "term_id": "GO:0051371",
  "gene_name": "PDZ and LIM domain protein 1"
}